{
  "term_id": "GO:0070120",
  "gene_symbol": "CNTFR",
  "gene": "UniProtKB:P26992",
  "gene_name": "Ciliary neurotrophic factor receptor subunit alpha",
  "term_label": "ciliary neurotrophic factor-mediated signaling pathway"
}